{
  "term_label": "positive regulation of cell-substrate adhesion",
  "gene_name": "Extracellular matrix protein 2",
  "gene_symbol": "ECM2",
  "gene": "UniProtKB:O94769",
  "term_id": "GO:0010811"
}